{
  "gene": "UniProtKB:P10275",
  "term_label": "male gonad development",
  "gene_name": "Androgen receptor",
  "term_id": "GO:0008584",
  "gene_symbol": "AR"
}